establishment of protein localization to peroxisome [GO:0072663] (biological process) Sources: GOC:mah Definition: The directed movement of a protein to a specific location in a peroxisome. Relationships: is a type of establishment of protein localization to organelle [GO:0072594] Subtypes: GO:0006625, protein import into peroxisome matrix [GO:0016558], protein import into peroxisome membrane [GO:0045046] Also known as: establishment of protein localisation to peroxisome